{
  "gene_name": "Group XIIB secretory phospholipase A2-like protein",
  "term_id": "GO:0070328",
  "gene": "UniProtKB:Q9BX93",
  "gene_symbol": "PLA2G12B",
  "term_label": "triglyceride homeostasis"
}